{
  "gene_name": "NADH dehydrogenase [ubiquinone] 1 beta subcomplex subunit 9",
  "term_id": "GO:0045271",
  "gene_symbol": "NDUFB9",
  "gene": "UniProtKB:Q9Y6M9",
  "term_label": "respiratory chain complex I"
}